{
  "gene_name": "Receptor-type tyrosine-protein phosphatase T",
  "term_label": "Unknown cellular component",
  "gene_symbol": "PTPRT",
  "term_id": "UNKNOWN:0003",
  "gene": "UniProtKB:O14522"
}